{
  "term_id": "GO:0007204",
  "gene_symbol": "CMKLR1",
  "term_label": "positive regulation of cytosolic calcium ion concentration",
  "gene": "UniProtKB:Q99788",
  "gene_name": "Chemerin-like receptor 1"
}